{
  "gene_name": "Fms-related tyrosine kinase 3 ligand",
  "term_label": "extracellular space",
  "term_id": "GO:0005615",
  "gene": "UniProtKB:P49771",
  "gene_symbol": "FLT3LG"
}